negative regulation of sarcinapterin biosynthetic process [GO:1900972] (BP) Definition: Any process that stops, prevents or reduces the frequency, rate or extent of sarcinapterin biosynthetic process. Relationships: is a type of GO:0009890; is a type of negative regulation of phosphate metabolic process [GO:0045936]; is a type of negative regulation of small molecule metabolic process [GO:0062014]; is a type of regulation of sarcinapterin biosynthetic process [GO:1900971]; negatively regulates GO:1900868 Sources: GOC:TermGenie, GOC:mengo_curators Also known as: down regulation of sarcinapterin anabolism, down regulation of sarcinapterin biosynthesis, down regulation of sarcinapterin biosynthetic process, down regulation of sarcinapterin formation, down regulation of sarcinapterin synthesis, down-regulation of sarcinapterin anabolism, down-regulation of sarcinapterin biosynthesis, down-regulation of sarcinapterin biosynthetic process, down-regulation of sarcinapterin formation, down-regulation of sarcinapterin synthesis, downregulation of sarcinapterin anabolism, downregulation of sarcinapterin biosynthesis, downregulation of sarcinapterin biosynthetic process, downregulation of sarcinapterin formation, downregulation of sarcinapterin synthesis, inhibition of sarcinapterin anabolism, inhibition of sarcinapterin biosynthesis, inhibition of sarcinapterin formation, inhibition of sarcinapterin synthesis, negative regulation of sarcinapterin anabolism, negative regulation of sarcinapterin biosynthesis, negative regulation of sarcinapterin formation, negative regulation of sarcinapterin synthesis, inhibition of sarcinapterin biosynthetic process